positive regulation of retinal rod cell fate commitment [GO:0060225] (biological process) Definition: Any process that increases the process in which the developmental fate of a cell becomes restricted such that it will develop into a retinal rod cell. A retinal rod cell is one of the two photoreceptor subtypes in a camera-type eye. Sources: GOC:dph Relationships: is a type of positive regulation of cell fate commitment [GO:0010455]; is a type of positive regulation of photoreceptor cell differentiation [GO:0046534]; is a type of regulation of retinal rod cell fate commitment [GO:0060224]; positively regulates retinal rod cell fate commitment [GO:0060223]